negative regulation of dopamine receptor signaling pathway [GO:0060160] (biological process) Definition: Any process that stops, prevents, or reduces the frequency, rate or extent of dopamine receptor protein signaling pathway activity. A dopamine receptor signaling pathway is the series of molecular signals generated as a consequence of a dopamine receptor binding to one of its physiological ligands. Sources: GOC:dph Relationships: is a type of negative regulation of G protein-coupled receptor signaling pathway [GO:0045744]; is a type of regulation of dopamine receptor signaling pathway [GO:0060159]; negatively regulates GO:0007212 Also known as: negative regulation of dopamine receptor signalling pathway Subtypes: negative regulation of phospholipase C-activating dopamine receptor signaling pathway [GO:0060162], negative regulation of adenylate cyclase-inhibiting dopamine receptor signaling pathway [GO:1904991]